{
  "gene_name": "GTP-binding protein 10",
  "term_label": "GTP binding",
  "gene_symbol": "GTPBP10",
  "gene": "UniProtKB:A4D1E9",
  "term_id": "GO:0005525"
}